ribonucleoside binding [GO:0032549] (molecular function) Relationships: is a type of nucleoside binding [GO:0001882] Subtypes: purine ribonucleoside binding [GO:0032550], GO:0032551 Sources: GOC:mah Definition: Binding to a ribonucleoside, a compound consisting of a purine or pyrimidine nitrogenous base linked to ribose.